{
  "gene_name": "Phosphatidylcholine:ceramide cholinephosphotransferase 1",
  "term_id": "GO:0000139",
  "gene_symbol": "SGMS1",
  "gene": "UniProtKB:Q86VZ5",
  "term_label": "Golgi membrane"
}